{
  "gene_name": "Leucine-rich repeat-containing protein 19",
  "gene_symbol": "LRRC19",
  "term_id": "GO:1901224",
  "gene": "UniProtKB:Q9H756",
  "term_label": "positive regulation of non-canonical NF-kappaB signal transduction"
}